{
  "term_id": "UNKNOWN:0003",
  "term_label": "Unknown cellular component",
  "gene": "UniProtKB:Q9Y2P0",
  "gene_symbol": "ZNF835",
  "gene_name": "Zinc finger protein 835"
}